{
  "gene_name": "Small ribosomal subunit protein uS11",
  "gene": "UniProtKB:P62263",
  "gene_symbol": "RPS14",
  "term_label": "translation",
  "term_id": "GO:0006412"
}